sphingolipid metabolic process [GO:0006665] (biological process) Definition: The chemical reactions and pathways involving sphingolipids, any of a class of lipids containing the long-chain amine diol sphingosine or a closely related base (a sphingoid). Sources: GOC:mah, ISBN:0198506732 Relationships: is_a membrane lipid metabolic process [GO:0006643] Subtypes: sphinganine-1-phosphate metabolic process [GO:0006668], GO:0006672, inositol phosphoceramide metabolic process [GO:0006673], sphingomyelin metabolic process [GO:0006684], glycosphingolipid metabolic process [GO:0006687], GO:0030148, sphingolipid catabolic process [GO:0030149], sphingoid metabolic process [GO:0046519] Also known as: sphingolipid metabolism